acroblast [GO:0036063] (cellular component) Also known as: spermatid acroblast Relationships: is a type of GO:0110165; BFO_0000050 GO:0005794 References: PMID:19934220 Sources: GOC:sart Definition: A cone-shaped structure in the head of a spermatozoon, which is formed by the coalescence of Golgi fragments following the completion of meiosis. The acroblast is situated adjacent to the acrosomal vesicle. Note: See also the fly_anatomy.ontology term 'acroblast ; FBbt:00004947'.